{
  "gene_name": "Polypeptide N-acetylgalactosaminyltransferase-like 6",
  "term_id": "GO:0006493",
  "gene_symbol": "GALNTL6",
  "term_label": "protein O-linked glycosylation",
  "gene": "UniProtKB:Q49A17"
}